{
  "gene_name": "Putative uncharacterized protein encoded by LINC00615",
  "term_id": "UNKNOWN:0001",
  "gene_symbol": "LINC00615",
  "gene": "UniProtKB:Q96LM1",
  "term_label": "Unknown molecular function"
}